{
  "gene": "UniProtKB:Q9UN67",
  "gene_name": "Protocadherin beta-10",
  "term_label": "plasma membrane",
  "term_id": "GO:0005886",
  "gene_symbol": "PCDHB10"
}